{
  "gene_symbol": "TNC",
  "gene": "UniProtKB:P24821",
  "gene_name": "Tenascin",
  "term_id": "GO:0030155",
  "term_label": "regulation of cell adhesion"
}